{
  "term_label": "transmitter-gated monoatomic ion channel activity involved in regulation of postsynaptic membrane potential",
  "gene_symbol": "GRID2",
  "gene_name": "Glutamate receptor ionotropic, delta-2",
  "gene": "UniProtKB:O43424",
  "term_id": "GO:1904315"
}